negative regulation of brain-derived neurotrophic factor receptor signaling pathway [GO:0031549] (biological process) Relationships: is a type of negative regulation of signal transduction [GO:0009968]; is a type of GO:0031548; negatively regulates brain-derived neurotrophic factor receptor signaling pathway [GO:0031547] Also known as: down regulation of brain-derived neurotrophic factor receptor signaling pathway, down-regulation of brain-derived neurotrophic factor receptor signaling pathway, downregulation of brain-derived neurotrophic factor receptor signaling pathway, negative regulation of BDNF receptor signaling pathway, negative regulation of BDNF receptor signalling pathway, negative regulation of brain-derived neurotrophic factor receptor signalling pathway, inhibition of brain-derived neurotrophic factor receptor signaling pathway Sources: GOC:mah Definition: Any process that stops, prevents, or reduces the frequency, rate or extent of signaling via the brain-derived neurotrophic factor receptor signaling pathway.